{
  "gene_name": "Putative keratin-associated protein 4-16",
  "term_id": "UNKNOWN:0003",
  "gene": "UniProtKB:G5E9R7",
  "gene_symbol": "KRTAP4-16",
  "term_label": "Unknown cellular component"
}